{
  "gene_name": "Inositol polyphosphate 5-phosphatase OCRL",
  "gene": "UniProtKB:Q01968",
  "term_label": "Unknown biological process",
  "term_id": "UNKNOWN:0002",
  "gene_symbol": "OCRL"
}